{
  "gene_name": "Ras-related protein Rab-6D",
  "gene_symbol": "RAB6D",
  "term_label": "GTPase activity",
  "term_id": "GO:0003924",
  "gene": "UniProtKB:Q53S08"
}